pulmonary artery morphogenesis [GO:0061156] (BP) Relationships: is a type of GO:0048844 Definition: The process in which the anatomical structures of the pulmonary artery are generated and organized. The pulmonary artery is the artery that carries blood from the heart to the lungs. Sources: GOC:dph, GOC:yaf